{
  "gene_symbol": "CLK2",
  "term_id": "GO:0043484",
  "term_label": "regulation of RNA splicing",
  "gene": "UniProtKB:P49760",
  "gene_name": "Dual specificity protein kinase CLK2"
}